{
  "gene_name": "Olfactory receptor 1J1",
  "gene": "UniProtKB:Q8NGS3",
  "term_id": "GO:0004984",
  "gene_symbol": "OR1J1",
  "term_label": "olfactory receptor activity"
}